{
  "term_id": "GO:0042571",
  "term_label": "immunoglobulin complex, circulating",
  "gene_name": "Immunoglobulin heavy constant alpha 2",
  "gene_symbol": "IGHA2",
  "gene": "UniProtKB:P01877"
}